{
  "gene_name": "Ras-related GTP-binding protein A",
  "term_label": "nucleus",
  "term_id": "GO:0005634",
  "gene": "UniProtKB:Q7L523",
  "gene_symbol": "RRAGA"
}